{
  "gene": "UniProtKB:Q5VSG8",
  "term_label": "Unknown cellular component",
  "gene_symbol": "MANEAL",
  "gene_name": "Glycoprotein endo-alpha-1,2-mannosidase-like protein",
  "term_id": "UNKNOWN:0003"
}